{
  "gene_name": "cAMP-dependent protein kinase catalytic subunit PRKX",
  "term_id": "GO:0007189",
  "term_label": "adenylate cyclase-activating G protein-coupled receptor signaling pathway",
  "gene_symbol": "PRKX",
  "gene": "UniProtKB:P51817"
}